{
  "term_id": "GO:0004984",
  "gene": "UniProtKB:Q8NGR5",
  "gene_name": "Olfactory receptor 1L4",
  "term_label": "olfactory receptor activity",
  "gene_symbol": "OR1L4"
}